{
  "gene": "UniProtKB:P0C8F1",
  "term_label": "Unknown molecular function",
  "term_id": "UNKNOWN:0001",
  "gene_symbol": "PATE4",
  "gene_name": "Prostate and testis expressed protein 4"
}